proteolysis within lysosome associated with antigen processing and presentation [GO:0002500] (biological process) Definition: The hydrolysis of a peptide bond or bonds within a protein by lysosomal resident proteases contributing to antigen processing and presentation. Relationships: is a type of proteolysis associated with antigen processing and presentation [GO:0002496]; occurs in lysosome [GO:0005764] References: PMID:15771591 Sources: GOC:add, ISBN:0781735149 Also known as: lysosomal proteolysis associated with antigen processing and presentation